regulation of adult salivary gland boundary specification [GO:0045707] (biological process) Relationships: is a type of regulation of salivary gland boundary specification [GO:0045704]; regulates adult salivary gland boundary specification [GO:0007434] Subtypes: negative regulation of adult salivary gland boundary specification [GO:0045709], GO:0045711 Sources: GOC:go_curators, GOC:tb Definition: Any process that modulates the frequency, rate or extent of salivary gland determination in an adult organism. Also known as: regulation of adult salivary gland determination